sister chromatid segregation [GO:0000819] (biological process) Definition: The cell cycle process in which sister chromatids are organized and then physically separated and apportioned to two or more sets. Relationships: is a type of chromosome organization [GO:0051276]; is a type of nuclear chromosome segregation [GO:0098813] Subtypes: mitotic sister chromatid segregation [GO:0000070], meiotic sister chromatid segregation [GO:0045144] Regulation: regulated by GO:0033045; negatively regulated by negative regulation of sister chromatid segregation [GO:0033046] Sources: GOC:ai, GOC:elh